{
  "gene": "UniProtKB:Q2Q1W2",
  "term_id": "GO:0043161",
  "gene_name": "E3 ubiquitin-protein ligase TRIM71",
  "gene_symbol": "TRIM71",
  "term_label": "proteasome-mediated ubiquitin-dependent protein catabolic process"
}